trans-zeatin O-beta-D-glucosyltransferase activity [GO:0050403] (molecular function) Definition: Catalysis of the reaction: trans-zeatin + UDP-D-glucose = O-beta-D-glucosyl-trans-zeatin + H+ + UDP. Sources: EC:2.4.1.203, RHEA:23224 Also known as: zeatin O-b-D-glucosyltransferase activity, UDP-glucose:trans-zeatin O-beta-D-glucosyltransferase activity, UDPglucose:trans-zeatin O-beta-D-glucosyltransferase activity, uridine diphosphoglucose-zeatin O-glucosyltransferase activity, zeatin O-beta-D-glucosyltransferase activity, zeatin O-glucosyltransferase activity Relationships: is a type of UDP-glucosyltransferase activity [GO:0035251]